{
  "gene_symbol": "OR52B4",
  "gene": "UniProtKB:Q8NGK2",
  "gene_name": "Olfactory receptor 52B4",
  "term_label": "Unknown biological process",
  "term_id": "UNKNOWN:0002"
}